{
  "gene_symbol": "FUT9",
  "gene": "UniProtKB:Q9Y231",
  "term_label": "Unknown biological process",
  "gene_name": "4-galactosyl-N-acetylglucosaminide 3-alpha-L-fucosyltransferase 9",
  "term_id": "UNKNOWN:0002"
}